{
  "gene_symbol": "MSR1",
  "gene_name": "Macrophage scavenger receptor types I and II",
  "term_label": "positive regulation of cholesterol storage",
  "term_id": "GO:0010886",
  "gene": "UniProtKB:P21757"
}